intermediate filament-based process [GO:0045103] (biological process) Relationships: is a type of cellular process [GO:0009987] Sources: GOC:ai Definition: Any cellular process that depends upon or alters the intermediate filament cytoskeleton, that part of the cytoskeleton comprising intermediate filaments and their associated proteins. Subtypes: intermediate filament cytoskeleton organization [GO:0045104]